{
  "term_label": "L-ascorbic acid metabolic process",
  "gene_symbol": "GSTO1",
  "gene_name": "Glutathione S-transferase omega-1",
  "term_id": "GO:0019852",
  "gene": "UniProtKB:P78417"
}